{
  "term_id": "GO:0005856",
  "gene": "UniProtKB:A0A140TA62",
  "gene_symbol": "LOC100653049",
  "term_label": "cytoskeleton",
  "gene_name": "IF rod domain-containing protein"
}